{
  "term_id": "GO:0000978",
  "term_label": "RNA polymerase II cis-regulatory region sequence-specific DNA binding",
  "gene_symbol": "KRBOX5",
  "gene_name": "KRAB domain-containing protein 5",
  "gene": "UniProtKB:Q7Z2F6"
}